hydroxyanthraquinone glucosyltransferase activity [GO:0047242] (molecular function) Sources: EC:2.4.1.181 Relationships: is a type of GO:0035251 Also known as: UDP-glucose:hydroxyanthraquinone O-glucosyltransferase activity, UDPglucose:hydroxyanthraquinone O-glucosyltransferase activity, anthraquinone-specific glucosyltransferase activity, uridine diphosphoglucose-anthraquinone glucosyltransferase activity Definition: Catalysis of the reaction: a hydroxyanthraquinone + UDP-D-glucose = a glucosyloxyanthraquinone + UDP.